{
  "term_label": "L-aspartate:2-oxoglutarate aminotransferase activity",
  "gene_symbol": "GOT1",
  "gene": "UniProtKB:P17174",
  "gene_name": "Aspartate aminotransferase, cytoplasmic",
  "term_id": "GO:0004069"
}